{
  "term_id": "GO:0016020",
  "term_label": "membrane",
  "gene": "UniProtKB:Q9BXB4",
  "gene_symbol": "OSBPL11",
  "gene_name": "Oxysterol-binding protein-related protein 11"
}